{
  "term_id": "GO:0071294",
  "gene_symbol": "MT1H",
  "gene_name": "Metallothionein-1H",
  "gene": "UniProtKB:P80294",
  "term_label": "cellular response to zinc ion"
}